{
  "gene_symbol": "IGHV3-49",
  "term_id": "GO:0003823",
  "term_label": "antigen binding",
  "gene_name": "Immunoglobulin heavy variable 3-49",
  "gene": "UniProtKB:A0A0A0MS15"
}